positive regulation of retrograde transport, endosome to Golgi [GO:1905281] (BP) Definition: Any process that activates or increases the frequency, rate or extent of retrograde transport, endosome to Golgi. Also known as: positive regulation of retrograde (endosome to Golgi) transport, up regulation of retrograde (endosome to Golgi) transport, up regulation of retrograde transport, endosome to Golgi, up-regulation of retrograde (endosome to Golgi) transport, up-regulation of retrograde transport, endosome to Golgi, upregulation of retrograde (endosome to Golgi) transport, upregulation of retrograde transport, endosome to Golgi, activation of retrograde (endosome to Golgi) transport, activation of retrograde transport, endosome to Golgi Relationships: is a type of GO:0032388; is a type of regulation of retrograde transport, endosome to Golgi [GO:1905279]; positively regulates retrograde transport, endosome to Golgi [GO:0042147] Sources: GOC:PARL, GOC:TermGenie, GOC:bf, GO_REF:0000058